{
  "gene_symbol": "CLMN",
  "gene_name": "Calmin",
  "gene": "UniProtKB:Q96JQ2",
  "term_label": "meiotic nuclear membrane microtubule tethering complex",
  "term_id": "GO:0034993"
}